{
  "gene_name": "Spindlin-1",
  "gene_symbol": "SPIN1",
  "gene": "UniProtKB:Q9Y657",
  "term_id": "GO:0005829",
  "term_label": "cytosol"
}